larval fat body development [GO:0007504] (biological process) Definition: The process whose specific outcome is the progression of the larval fat body over time, from its formation to the mature structure. The larval fat body consists of a bilaterally symmetrical monolayer of cells lying between the gut and the muscles of the body wall. As in other tissues of the larva, the cells of the fat body complete their divisions in the embryo and increase in size and ploidy during larval life. Relationships: is a type of fat body development [GO:0007503]; is part of GO:0002168 Sources: GOC:bf, ISBN:0879694238